{
  "gene": "UniProtKB:P23471",
  "gene_name": "Receptor-type tyrosine-protein phosphatase zeta",
  "gene_symbol": "PTPRZ1",
  "term_label": "oligodendrocyte differentiation",
  "term_id": "GO:0048709"
}